{
  "gene": "UniProtKB:P17017",
  "gene_name": "Zinc finger protein 14",
  "gene_symbol": "ZNF14",
  "term_id": "GO:0000977",
  "term_label": "RNA polymerase II transcription regulatory region sequence-specific DNA binding"
}